{
  "gene_name": "Calcium-activated potassium channel subunit beta-1",
  "gene_symbol": "KCNMB1",
  "term_id": "GO:0008076",
  "gene": "UniProtKB:Q16558",
  "term_label": "voltage-gated potassium channel complex"
}